{
  "term_id": "GO:0045892",
  "gene": "UniProtKB:Q14135",
  "gene_name": "Transcription cofactor vestigial-like protein 4",
  "gene_symbol": "VGLL4",
  "term_label": "negative regulation of DNA-templated transcription"
}